microtubule site clamp [GO:1990644] (molecular function) Relationships: is a type of protein-macromolecule adaptor activity [GO:0030674] References: PMID:20723757 Definition: The binding activity of a molecule that attaches the spindle microtubules to the kinetochore.